{
  "gene": "UniProtKB:Q58EX7",
  "gene_name": "Puratrophin-1",
  "gene_symbol": "PLEKHG4",
  "term_label": "cytoplasm",
  "term_id": "GO:0005737"
}